{
  "term_id": "GO:0005634",
  "gene_symbol": "H2AP",
  "gene": "UniProtKB:O75409",
  "term_label": "nucleus",
  "gene_name": "Huntingtin-interacting protein M"
}